{
  "term_id": "GO:0005886",
  "term_label": "plasma membrane",
  "gene": "UniProtKB:A6NND4",
  "gene_name": "Olfactory receptor 2AT4",
  "gene_symbol": "OR2AT4"
}